{
  "term_label": "Unknown molecular function",
  "term_id": "UNKNOWN:0001",
  "gene_symbol": "TMEM269",
  "gene_name": "Transmembrane protein 269",
  "gene": "UniProtKB:A0A1B0GVZ9"
}